{
  "term_id": "GO:0015629",
  "term_label": "actin cytoskeleton",
  "gene_name": "Leucine zipper protein 1",
  "gene": "UniProtKB:Q86V48",
  "gene_symbol": "LUZP1"
}